6-phospho-beta-galactosidase activity [GO:0033920] (molecular function) Definition: Catalysis of the reaction: a 6-phospho-beta-D-galactoside + H2O = 6-phospho-D-galactose + an alcohol. Also known as: 6-phospho-beta-D-galactosidase activity, 6-phospho-beta-D-galactoside 6-phosphogalactohydrolase activity, beta-D-phosphogalactoside galactohydrolase activity, phospho-beta-D-galactosidase activity, phospho-beta-galactosidase activity Relationships: is a type of galactosidase activity [GO:0015925] Sources: RHEA:24568